{
  "gene_symbol": "GPR137",
  "gene_name": "Integral membrane protein GPR137",
  "gene": "UniProtKB:Q96N19",
  "term_id": "GO:1904263",
  "term_label": "positive regulation of TORC1 signaling"
}